{
  "term_id": "GO:0004596",
  "term_label": "protein-N-terminal amino-acid acetyltransferase activity",
  "gene_name": "N-alpha-acetyltransferase 80",
  "gene_symbol": "NAA80",
  "gene": "UniProtKB:Q93015"
}